{
  "gene": "UniProtKB:Q9BZ97",
  "gene_name": "Putative transcript Y 13 protein",
  "term_id": "UNKNOWN:0002",
  "gene_symbol": "TTTY13",
  "term_label": "Unknown biological process"
}